{
  "term_label": "Unknown cellular component",
  "term_id": "UNKNOWN:0003",
  "gene_symbol": "TMEM54",
  "gene_name": "Transmembrane protein 54",
  "gene": "UniProtKB:Q969K7"
}